{
  "term_label": "plasma membrane",
  "gene": "UniProtKB:Q9H3T2",
  "gene_symbol": "SEMA6C",
  "gene_name": "Semaphorin-6C",
  "term_id": "GO:0005886"
}